{
  "term_id": "GO:0046329",
  "gene_symbol": "DUSP3",
  "term_label": "negative regulation of JNK cascade",
  "gene_name": "Dual specificity protein phosphatase 3",
  "gene": "UniProtKB:P51452"
}